{
  "term_label": "beta-N-acetylhexosaminidase activity",
  "gene": "UniProtKB:P06865",
  "gene_name": "Beta-hexosaminidase subunit alpha",
  "term_id": "GO:0004563",
  "gene_symbol": "HEXA"
}